{
  "gene_name": "Acylglycerol kinase, mitochondrial",
  "term_label": "ceramide kinase activity",
  "gene_symbol": "AGK",
  "gene": "UniProtKB:Q53H12",
  "term_id": "GO:0001729"
}